{
  "gene_name": "Transforming protein RhoA",
  "term_id": "GO:0043149",
  "term_label": "stress fiber assembly",
  "gene_symbol": "RHOA",
  "gene": "UniProtKB:P61586"
}